{
  "term_id": "GO:0005737",
  "gene": "UniProtKB:Q9C0H6",
  "gene_name": "Kelch-like protein 4",
  "gene_symbol": "KLHL4",
  "term_label": "cytoplasm"
}